{
  "gene": "UniProtKB:P12838",
  "term_id": "GO:0051673",
  "term_label": "disruption of plasma membrane integrity in another organism",
  "gene_name": "Defensin alpha 4",
  "gene_symbol": "DEFA4"
}